{
  "gene": "UniProtKB:P46089",
  "term_id": "GO:0005886",
  "gene_symbol": "GPR3",
  "gene_name": "G-protein coupled receptor 3",
  "term_label": "plasma membrane"
}